{
  "term_id": "GO:0007268",
  "gene_name": "D(4) dopamine receptor",
  "gene_symbol": "DRD4",
  "term_label": "chemical synaptic transmission",
  "gene": "UniProtKB:P21917"
}